beta-alanyl-histamine hydrolase activity [GO:0031964] (molecular function) Definition: Catalysis of the reaction: carcinine + H2O = histamine + beta-alanine. Carcinine is also known as N-beta-alanyl histamine. Also known as: carcinine hydrolase activity Relationships: is a type of hydrolase activity, acting on carbon-nitrogen (but not peptide) bonds, in linear amides [GO:0016811] References: PMID:16299587 Sources: RHEA:73463